Golgi vesicle transport [GO:0048193] (biological process) Definition: The directed movement of substances into, out of or within the Golgi apparatus, mediated by vesicles. References: PMID:10219233 Sources: GOC:jid, ISBN:0716731363 Also known as: Golgi-derived vesicle transport Relationships: is a type of vesicle-mediated transport [GO:0016192] Subtypes: GO:0006888, retrograde vesicle-mediated transport, Golgi to endoplasmic reticulum [GO:0006890], intra-Golgi vesicle-mediated transport [GO:0006891], post-Golgi vesicle-mediated transport [GO:0006892], early endosome to Golgi transport [GO:0034498], GO:0034499, recycling endosome to Golgi transport [GO:0071955]